{
  "gene_name": "E3 ubiquitin-protein ligase TRIM71",
  "gene_symbol": "TRIM71",
  "gene": "UniProtKB:Q2Q1W2",
  "term_id": "GO:0000932",
  "term_label": "P-body"
}